{
  "gene_symbol": "ENOX1",
  "gene": "UniProtKB:Q8TC92",
  "gene_name": "Ecto-NOX disulfide-thiol exchanger 1",
  "term_label": "Unknown biological process",
  "term_id": "UNKNOWN:0002"
}